regulation of collateral sprouting of injured axon [GO:0048693] (biological process) Relationships: is a type of regulation of collateral sprouting [GO:0048670]; is a type of regulation of sprouting of injured axon [GO:0048686]; regulates GO:0048674 Subtypes: positive regulation of collateral sprouting of injured axon [GO:0048694], negative regulation of collateral sprouting of injured axon [GO:0048695] Sources: GOC:dgh, GOC:dph, GOC:jid, GOC:lm Definition: Any process that modulates the frequency, rate or extent of collateral sprouting of an injured axon.